acetylornithine deacetylase activity [GO:0008777] (molecular function) Relationships: is a type of GO:0016811; is a type of deacetylase activity [GO:0019213] Sources: EC:3.5.1.16 Also known as: N-acetylornithinase activity, acetylornithinase activity, 2-N-acetyl-L-ornithine amidohydrolase activity, N2-acetyl-L-ornithine amidohydrolase activity Definition: Catalysis of the reaction: N2-acetyl-L-ornithine + H2O = acetate + L-ornithine.